nucleobase transport [GO:0015851] (biological process) Definition: The directed movement of a nucleobase, any nitrogenous base that is a constituent of a nucleoside, nucleotide, or nucleic acid, into, out of or within a cell, or between cells, by means of some agent such as a transporter or pore. Subtypes: purine nucleobase transport [GO:0006863], pyrimidine nucleobase transport [GO:0015855] Also known as: nucleobase transmembrane transport Sources: ISBN:0198506732 Relationships: is a type of nitrogen compound transport [GO:0071705]